{
  "term_id": "GO:0031490",
  "term_label": "chromatin DNA binding",
  "gene": "UniProtKB:Q969T9",
  "gene_symbol": "WBP2",
  "gene_name": "WW domain-binding protein 2"
}